{
  "gene": "UniProtKB:P29803",
  "gene_name": "Pyruvate dehydrogenase E1 component subunit alpha, testis-specific form, mitochondrial",
  "term_id": "GO:0006086",
  "term_label": "pyruvate decarboxylation to acetyl-CoA",
  "gene_symbol": "PDHA2"
}